peptidyl-tyrosine autophosphorylation [GO:0038083] (biological process) Definition: The phosphorylation by a protein of one or more of its own tyrosine amino acid residues, or a tyrosine residue on an identical protein. Also known as: tyrosine autophosphorylation, RTK autophosphorylation, receptor tyrosine kinase autophosphorylation Relationships: is a type of peptidyl-tyrosine phosphorylation [GO:0018108]; is a type of protein autophosphorylation [GO:0046777] References: PMID:10037737, PMID:10068444, PMID:10940390 Regulation: regulated by regulation of peptidyl-tyrosine autophosphorylation [GO:1900084]; negatively regulated by negative regulation of peptidyl-tyrosine autophosphorylation [GO:1900085]; positively regulated by positive regulation of peptidyl-tyrosine autophosphorylation [GO:1900086]